{
  "gene_name": "Olfactory receptor 10R2",
  "gene_symbol": "OR10R2",
  "term_label": "membrane",
  "term_id": "GO:0016020",
  "gene": "UniProtKB:Q8NGX6"
}